chloroplast thylakoid [GO:0009534] (CC) Definition: Sac-like membranous structures (cisternae) in a chloroplast combined into stacks (grana) and present singly in the stroma (stroma thylakoids or frets) as interconnections between grana. An example of this component is found in Arabidopsis thaliana. Sources: GOC:mtg_sensu, ISBN:0943088399 Relationships: is a type of plastid thylakoid [GO:0031976]; is part of chloroplast [GO:0009507] Subtypes: granal stacked thylakoid [GO:0009515], chloroplast stromal thylakoid [GO:0009533]